{
  "gene_name": "KAT8 regulatory NSL complex subunit 1",
  "term_id": "UNKNOWN:0002",
  "gene": "UniProtKB:Q7Z3B3",
  "term_label": "Unknown biological process",
  "gene_symbol": "KANSL1"
}